{
  "term_id": "GO:0004090",
  "gene_name": "Carbonyl reductase [NADPH] 1",
  "gene_symbol": "CBR1",
  "gene": "UniProtKB:P16152",
  "term_label": "carbonyl reductase (NADPH) activity"
}